polygalacturonase inhibitor activity [GO:0090353] (MF) Sources: GOC:tb Relationships: is a type of GO:0004857; negatively regulates polygalacturonase activity [GO:0004650] Definition: Binds to and stops, prevents or reduces the activity of polygalacturonase.